{
  "gene_symbol": "DNAJB2",
  "gene_name": "DnaJ homolog subfamily B member 2",
  "term_label": "Hsp70 protein binding",
  "term_id": "GO:0030544",
  "gene": "UniProtKB:P25686"
}